regulation of DNA recombinase mediator complex assembly [GO:1903872] (biological process) Subtypes: GO:1903873 Relationships: is a type of regulation of protein-containing complex assembly [GO:0043254]; regulates DNA recombinase mediator complex assembly [GO:1903871] References: PMID:18347097 Sources: GOC:TermGenie, GOC:rb, GO_REF:0000058 Also known as: regulation of DNA recombinase mediator complex formation Definition: Any process that modulates the frequency, rate or extent of DNA recombinase mediator complex assembly.